{
  "term_id": "GO:0005634",
  "gene": "UniProtKB:Q8WUA2",
  "gene_name": "Peptidyl-prolyl cis-trans isomerase-like 4",
  "gene_symbol": "PPIL4",
  "term_label": "nucleus"
}